{
  "term_label": "L-glutamine transmembrane transporter activity",
  "gene_symbol": "SLC38A1",
  "term_id": "GO:0015186",
  "gene": "UniProtKB:Q9H2H9",
  "gene_name": "Sodium-coupled neutral amino acid symporter 1"
}